{
  "gene": "UniProtKB:Q5MJ08",
  "gene_name": "Sperm protein associated with the nucleus on the X chromosome N4",
  "term_id": "UNKNOWN:0002",
  "term_label": "Unknown biological process",
  "gene_symbol": "SPANXN4"
}